{
  "gene_symbol": "SLC25A24",
  "term_label": "ATP transport",
  "gene_name": "Mitochondrial adenyl nucleotide antiporter SLC25A24",
  "gene": "UniProtKB:Q6NUK1",
  "term_id": "GO:0015867"
}